{
  "gene_name": "Interleukin-22 receptor subunit alpha-1",
  "term_label": "cytokine-mediated signaling pathway",
  "gene": "UniProtKB:Q8N6P7",
  "term_id": "GO:0019221",
  "gene_symbol": "IL22RA1"
}